{
  "gene_name": "Prominin-2",
  "term_id": "UNKNOWN:0001",
  "term_label": "Unknown molecular function",
  "gene_symbol": "PROM2",
  "gene": "UniProtKB:Q8N271"
}